{
  "term_label": "endosome",
  "term_id": "GO:0005768",
  "gene_symbol": "SNX1",
  "gene_name": "Sorting nexin-1",
  "gene": "UniProtKB:Q13596"
}